{
  "term_id": "GO:0000981",
  "gene": "UniProtKB:Q8TBZ5",
  "term_label": "DNA-binding transcription factor activity, RNA polymerase II-specific",
  "gene_name": "Zinc finger protein 502",
  "gene_symbol": "ZNF502"
}